{
  "term_id": "GO:0044877",
  "gene_symbol": "NUF2",
  "gene_name": "Kinetochore protein Nuf2",
  "gene": "UniProtKB:Q9BZD4",
  "term_label": "protein-containing complex binding"
}